{
  "term_id": "UNKNOWN:0001",
  "gene_name": "Membrane-spanning 4-domains subfamily A member 8",
  "gene_symbol": "MS4A8",
  "term_label": "Unknown molecular function",
  "gene": "UniProtKB:Q9BY19"
}